{
  "gene": "UniProtKB:Q9Y496",
  "gene_name": "Kinesin-like protein KIF3A",
  "term_label": "ATP hydrolysis activity",
  "term_id": "GO:0016887",
  "gene_symbol": "KIF3A"
}